{
  "gene_name": "Actin-related protein 5",
  "gene_symbol": "ACTR5",
  "term_id": "GO:0030234",
  "term_label": "enzyme regulator activity",
  "gene": "UniProtKB:Q9H9F9"
}